trans-cinnamate 2-monooxygenase activity [GO:0050344] (molecular function) Sources: EC:1.14.13.14, RHEA:10956 Relationships: is a type of GO:0016709 Definition: Catalysis of the reaction: trans-cinnamate + H+ + NADPH + O2 = 2-coumarate + H2O + NADP+. Also known as: trans-cinnamic acid 2-hydroxylase activity, cinnamate 2-hydroxylase activity, cinnamate 2-monooxygenase activity, cinnamic 2-hydroxylase activity, cinnamic acid 2-hydroxylase activity, trans-cinnamate,NADPH:oxygen oxidoreductase (2-hydroxylating)